polychlorinated biphenyl binding [GO:0097160] (molecular function) Definition: Binding to a polychlorinated biphenyl (PCB), a biphenyl compound containing between 2 and 10 chlorine atoms attached to the two benzene rings. References: PMID:7583672 Sources: GOC:sjw Also known as: PCB binding, polychlorobiphenyl binding Relationships: is a type of binding [GO:0005488]